{
  "gene_name": "Elongation of very long chain fatty acids protein 5",
  "gene": "UniProtKB:Q9NYP7",
  "term_id": "GO:0030148",
  "gene_symbol": "ELOVL5",
  "term_label": "sphingolipid biosynthetic process"
}